tectospinal tract morphogenesis [GO:0021977] (biological process) Relationships: is a type of central nervous system projection neuron axonogenesis [GO:0021952] Sources: GOC:cls, GOC:dgh, GOC:dph, GOC:jid, GO_REF:0000021 Definition: Generation of a long process of a CNS neuron, that carries efferent (outgoing) action potentials from the cell body in the superior colliculus of the midbrain towards target cells in the ventral spinal cord.